phytoene dehydrogenase activity [GO:0016166] (molecular function) Relationships: is a type of oxidoreductase activity, acting on the CH-CH group of donors [GO:0016627] Definition: Catalysis of the dehydrogenation of phytoene to produce a carotenoid intermediate such as phytofluene. References: PMID:29176862